relaxation of cardiac muscle [GO:0055119] (biological process) Definition: The process in which the extent of cardiac muscle contraction is reduced. Regulation: regulated by regulation of relaxation of cardiac muscle [GO:1901897]; negatively regulated by negative regulation of relaxation of cardiac muscle [GO:1901898]; positively regulated by positive regulation of relaxation of cardiac muscle [GO:1901899] Sources: GOC:ecd Relationships: is a type of relaxation of muscle [GO:0090075]